actin filament-based process [GO:0030029] (biological process) Definition: Any cellular process that depends upon or alters the actin cytoskeleton, that part of the cytoskeleton comprising actin filaments and their associated proteins. Sources: GOC:mah Regulation: regulated by regulation of actin filament-based process [GO:0032970] Subtypes: GO:0030036, GO:0030048, actin filament severing [GO:0051014], protein localization involved in acrosome reaction [GO:0060476] Also known as: microfilament-based process Relationships: is a type of cellular process [GO:0009987]